{
  "gene_name": "Proline-rich protein, Y-linked",
  "term_label": "Unknown molecular function",
  "gene": "UniProtKB:Q9H606",
  "term_id": "UNKNOWN:0001",
  "gene_symbol": "PRORY"
}